{
  "gene_name": "Hydrocephalus-inducing protein homolog",
  "term_id": "UNKNOWN:0001",
  "gene_symbol": "HYDIN",
  "term_label": "Unknown molecular function",
  "gene": "UniProtKB:Q4G0P3"
}